{
  "gene_name": "F-box_WD repeat-containing protein 11",
  "term_label": "microtubule organizing center organization",
  "gene": "UniProtKB:Q9UKB1",
  "term_id": "GO:0031023",
  "gene_symbol": "FBXW11"
}